nuclease inhibitor activity [GO:0140721] (molecular function) Subtypes: ribonuclease inhibitor activity [GO:0008428], deoxyribonuclease inhibitor activity [GO:0060703] Relationships: is_a enzyme inhibitor activity [GO:0004857]; negatively regulates nuclease activity [GO:0004518] References: PMID:28785032, PMID:29554913, PMID:30046034 Definition: Binds to and modulates the activity of a nuclease.